ovulation cycle process [GO:0022602] (biological process) Definition: A process involved in the sexual cycle seen in females, often with physiologic changes in the endometrium that recur at regular intervals during the reproductive years. Sources: GOC:isa_complete Also known as: estrous cycle process, menstrual cycle process Relationships: is a type of reproductive process [GO:0022414]; is a type of rhythmic process [GO:0048511]; is part of ovulation cycle [GO:0042698] Subtypes: GO:0001542, GO:0001543, initiation of primordial ovarian follicle growth [GO:0001544], GO:0001545, preantral ovarian follicle growth [GO:0001546], GO:0001547, follicular fluid formation in ovarian follicle antrum [GO:0001548], ovarian cumulus expansion [GO:0001550], ovarian follicle endowment [GO:0001551], luteinization [GO:0001553], luteolysis [GO:0001554], GO:0042699, progesterone secretion [GO:0042701], uterine wall growth [GO:0042702], uterine wall breakdown [GO:0042704], generation of ovulation cycle rhythm [GO:0060112]